{
  "term_label": "cellular response to type II interferon",
  "gene_name": "Guanylate-binding protein 1",
  "gene_symbol": "GBP1",
  "gene": "UniProtKB:P32455",
  "term_id": "GO:0071346"
}